{
  "gene_symbol": "ZNRF2",
  "term_label": "cytoplasm",
  "term_id": "GO:0005737",
  "gene_name": "E3 ubiquitin-protein ligase ZNRF2",
  "gene": "UniProtKB:Q8NHG8"
}